{
  "gene_symbol": "RNF225",
  "gene_name": "RING finger protein 225",
  "gene": "UniProtKB:M0QZC1",
  "term_id": "GO:0061630",
  "term_label": "ubiquitin protein ligase activity"
}